{
  "gene_symbol": "RPL19",
  "gene": "UniProtKB:P84098",
  "term_id": "GO:0003723",
  "term_label": "RNA binding",
  "gene_name": "Large ribosomal subunit protein eL19"
}